{
  "gene_symbol": "ATP6V1G1",
  "term_label": "Unknown molecular function",
  "gene": "UniProtKB:O75348",
  "term_id": "UNKNOWN:0001",
  "gene_name": "V-type proton ATPase subunit G 1"
}